norepinephrine secretion, neurotransmission [GO:0061533] (biological process) Relationships: is a type of norepinephrine secretion [GO:0048243]; is a type of GO:0160043 Also known as: noradrenaline secretion, neurotransmission Definition: The regulated release of norepinephrine by a cell, in which the norepinephrine acts as a neurotransmitter. Sources: GOC:dph